{
  "gene_name": "Uncharacterized protein",
  "term_id": "UNKNOWN:0003",
  "gene_symbol": "Q6YL49",
  "gene": "UniProtKB:Q6YL49",
  "term_label": "Unknown cellular component"
}